{
  "term_id": "GO:0005686",
  "gene": "UniProtKB:Q7RTV0",
  "term_label": "U2 snRNP",
  "gene_name": "PHD finger-like domain-containing protein 5A",
  "gene_symbol": "PHF5A"
}